{
  "gene_name": "Ubiquitin carboxyl-terminal hydrolase CYLD",
  "term_id": "GO:0005829",
  "term_label": "cytosol",
  "gene_symbol": "CYLD",
  "gene": "UniProtKB:Q9NQC7"
}